negative regulation of smooth muscle cell migration [GO:0014912] (biological process) Relationships: is a type of regulation of smooth muscle cell migration [GO:0014910]; is a type of negative regulation of cell migration [GO:0030336]; negatively regulates smooth muscle cell migration [GO:0014909] Sources: CL:0000192, GOC:mtg_muscle Subtypes: GO:0071672, negative regulation of vascular associated smooth muscle cell migration [GO:1904753] Definition: Any process that stops, prevents, or reduces the frequency, rate or extent of smooth muscle cell migration.